{
  "gene": "UniProtKB:Q9P0V9",
  "gene_name": "Septin-10",
  "term_id": "GO:0003924",
  "gene_symbol": "SEPTIN10",
  "term_label": "GTPase activity"
}